{
  "term_label": "aminophospholipid flippase activity",
  "gene_name": "Cell cycle control protein 50A",
  "gene_symbol": "TMEM30A",
  "term_id": "GO:0015247",
  "gene": "UniProtKB:Q9NV96"
}